ascorbate homeostasis [GO:0140576] (biological process) Also known as: cellular ascorbate homeostasis Definition: Any process involved in the maintenance of an internal steady state of ascorbate at the level of a cell. Relationships: is a type of chemical homeostasis [GO:0048878] References: PMID:1623014, PMID:17068337, PMID:32547589